{
  "gene_symbol": "TRRAP",
  "term_id": "GO:0006355",
  "gene": "UniProtKB:Q9Y4A5",
  "term_label": "regulation of DNA-templated transcription",
  "gene_name": "Transformation_transcription domain-associated protein"
}